positive regulation of angiogenesis [GO:0045766] (BP) Relationships: is a type of GO:0045765; is a type of GO:1904018; positively regulates angiogenesis [GO:0001525] Definition: Any process that activates or increases angiogenesis. Also known as: up regulation of angiogenesis, up-regulation of angiogenesis, upregulation of angiogenesis, activation of angiogenesis, stimulation of angiogenesis Subtypes: positive regulation of vascular wound healing [GO:0035470], positive regulation of sprouting angiogenesis [GO:1903672], positive regulation of blood vessel branching [GO:1905555] Sources: GOC:go_curators